host cell endoplasmic reticulum-Golgi intermediate compartment membrane [GO:0044173] (cellular component) Sources: GOC:jl Also known as: host ER-Golgi intermediate compartment membrane, host cell ER-Golgi intermediate compartment membrane, host endoplasmic reticulum-Golgi intermediate compartment membrane Relationships: is a type of host cell membrane [GO:0033644]; is part of host cell endoplasmic reticulum-Golgi intermediate compartment [GO:0044172] Definition: The lipid bilayer surrounding any of the compartments of the host cell ER-Golgi intermediate compartment system.